{
  "gene": "UniProtKB:Q96RJ0",
  "gene_symbol": "TAAR1",
  "term_id": "GO:0005886",
  "gene_name": "Trace amine-associated receptor 1",
  "term_label": "plasma membrane"
}